{
  "gene_symbol": "GBX1",
  "term_id": "GO:0006357",
  "gene": "UniProtKB:Q14549",
  "term_label": "regulation of transcription by RNA polymerase II",
  "gene_name": "Homeobox protein GBX-1"
}